{
  "term_id": "GO:0003729",
  "gene_name": "Developmental pluripotency-associated 5 protein",
  "gene": "UniProtKB:A6NC42",
  "term_label": "mRNA binding",
  "gene_symbol": "DPPA5"
}